{
  "term_label": "Unknown molecular function",
  "gene_name": "Putative uncharacterized protein encoded by LINC00315",
  "term_id": "UNKNOWN:0001",
  "gene_symbol": "LINC00315",
  "gene": "UniProtKB:P59091"
}